{
  "term_id": "GO:0005634",
  "gene": "UniProtKB:Q9BRH9",
  "term_label": "nucleus",
  "gene_symbol": "ZNF251",
  "gene_name": "Zinc finger protein 251"
}